{
  "gene_name": "Myosin light chain kinase 3",
  "gene": "UniProtKB:Q32MK0",
  "term_id": "GO:0015629",
  "term_label": "actin cytoskeleton",
  "gene_symbol": "MYLK3"
}